{
  "gene_name": "A-kinase anchor protein 8-like",
  "gene": "UniProtKB:Q9ULX6",
  "term_id": "GO:0034237",
  "term_label": "protein kinase A regulatory subunit binding",
  "gene_symbol": "AKAP8L"
}